{
  "gene_name": "Target of rapamycin complex 2 subunit MAPKAP1",
  "term_id": "GO:0005737",
  "gene": "UniProtKB:Q9BPZ7",
  "gene_symbol": "MAPKAP1",
  "term_label": "cytoplasm"
}